{
  "term_label": "cytoplasm",
  "gene_name": "5'-deoxynucleotidase HDDC2",
  "gene": "UniProtKB:Q7Z4H3",
  "gene_symbol": "HDDC2",
  "term_id": "GO:0005737"
}